imitative learning [GO:0098596] (biological process) Relationships: is a type of observational learning [GO:0098597] Sources: GOC:dos, Wikipedia:Imitative_learning&oldid=593192364 Definition: Learning in which new behaviors are acquired through imitation. Subtypes: vocal learning [GO:0042297]